{
  "gene_symbol": "KLF6",
  "gene": "UniProtKB:Q99612",
  "gene_name": "Krueppel-like factor 6",
  "term_label": "DNA-binding transcription factor activity, RNA polymerase II-specific",
  "term_id": "GO:0000981"
}